{
  "gene_name": "Enhancer of polycomb homolog 2",
  "gene_symbol": "EPC2",
  "gene": "UniProtKB:Q52LR7",
  "term_id": "GO:0006357",
  "term_label": "regulation of transcription by RNA polymerase II"
}